{
  "term_id": "GO:0005635",
  "term_label": "nuclear envelope",
  "gene_symbol": "CHMP4BP1",
  "gene_name": "Putative charged multivesicular body protein 4B-like protein CHMP4BP1",
  "gene": "UniProtKB:P59074"
}